{
  "gene_name": "Rho-related GTP-binding protein RhoQ",
  "term_label": "protein kinase binding",
  "gene_symbol": "RHOQ",
  "gene": "UniProtKB:P17081",
  "term_id": "GO:0019901"
}